{
  "term_id": "UNKNOWN:0001",
  "term_label": "Unknown molecular function",
  "gene": "UniProtKB:Q7Z6M1",
  "gene_symbol": "RABEPK",
  "gene_name": "Rab9 effector protein with kelch motifs"
}